{
  "gene": "UniProtKB:P40763",
  "term_label": "nucleus",
  "gene_name": "Signal transducer and activator of transcription 3",
  "term_id": "GO:0005634",
  "gene_symbol": "STAT3"
}